{
  "term_label": "RNA binding",
  "term_id": "GO:0003723",
  "gene_symbol": "RPS4Y2",
  "gene": "UniProtKB:Q8TD47",
  "gene_name": "Small ribosomal subunit protein eS4, Y isoform 2"
}